11-oxo-beta-amyrin 30-oxidase activity [GO:0102375] (molecular function) Definition: Catalysis of the reaction: 11-oxo-beta-amyrin + 3 NADPH + 3 O2 + 2 H+ = glycyrrhetinic acid + 3 NADP + 4 H2O. Relationships: is_a GO:0016709 Sources: GOC:pz, RHEA:35499